{
  "term_label": "protein-macromolecule adaptor activity",
  "gene": "UniProtKB:Q5MNZ6",
  "gene_name": "WD repeat domain phosphoinositide-interacting protein 3",
  "term_id": "GO:0030674",
  "gene_symbol": "WDR45B"
}